{
  "gene": "UniProtKB:P06748",
  "term_label": "ribosomal small subunit export from nucleus",
  "gene_name": "Nucleophosmin",
  "term_id": "GO:0000056",
  "gene_symbol": "NPM1"
}